{
  "term_id": "GO:0005737",
  "term_label": "cytoplasm",
  "gene_name": "Ret finger protein-like 4A",
  "gene_symbol": "RFPL4A",
  "gene": "UniProtKB:A6NLU0"
}